glucan 1,4-alpha-maltohydrolase activity [GO:0043897] (molecular function) Definition: Catalysis of the hydrolysis of (1->4)-alpha-D-glucosidic linkages in polysaccharides so as to remove successive alpha-maltose residues from the non-reducing ends of the chains. Sources: EC:3.2.1.133 Also known as: 1,4-alpha-D-glucan alpha-maltohydrolase activity, glucan-1,4-alpha-maltohydrolase activity, maltogenic alpha-amylase activity Relationships: is a type of hydrolase activity, hydrolyzing O-glycosyl compounds [GO:0004553]